{
  "gene_name": "Cysteine protease ATG4C",
  "gene_symbol": "ATG4C",
  "term_label": "aggrephagy",
  "gene": "UniProtKB:Q96DT6",
  "term_id": "GO:0035973"
}